{
  "gene_symbol": "ERBB3",
  "term_id": "GO:0007173",
  "gene": "UniProtKB:P21860",
  "term_label": "epidermal growth factor receptor signaling pathway",
  "gene_name": "Receptor tyrosine-protein kinase erbB-3"
}